coagulation [GO:0050817] (biological process) Sources: ISBN:0198506732 Subtypes: blood coagulation [GO:0007596], GO:0042381 Definition: The process in which a fluid solution, or part of it, changes into a solid or semisolid mass. Also known as: clotting Relationships: is a type of multicellular organismal process [GO:0032501] Regulation: regulated by regulation of coagulation [GO:0050818]; negatively regulated by negative regulation of coagulation [GO:0050819]; positively regulated by positive regulation of coagulation [GO:0050820]